{
  "gene_name": "Ovarian cancer G-protein coupled receptor 1",
  "gene_symbol": "GPR68",
  "term_label": "Unknown cellular component",
  "term_id": "UNKNOWN:0003",
  "gene": "UniProtKB:Q15743"
}